{
  "gene_symbol": "DNAH14",
  "term_id": "GO:0051959",
  "gene_name": "Dynein axonemal heavy chain 14",
  "term_label": "dynein light intermediate chain binding",
  "gene": "UniProtKB:Q0VDD8"
}